alkylglycerone-phosphate synthase activity [GO:0008609] (molecular function) Relationships: is a type of transferase activity, transferring alkyl or aryl (other than methyl) groups [GO:0016765] Sources: EC:2.5.1.26 Also known as: 1-acyl-glycerone-3-phosphate:long-chain-alcohol O-3-phospho-2-oxopropanyltransferase activity, DHAP-AT, alkyl DHAP synthetase activity, alkyl-DHAP, alkyl-DHAP synthase activity, alkyldihydroxyacetone phosphate synthetase activity, alkyldihydroxyacetonephosphate synthase activity, dihydroxyacetone-phosphate acyltransferase activity Definition: Catalysis of the reaction: 1-acyl-glycerone 3-phosphate + a long-chain alcohol = 1-alkyl-glycerone 3-phosphate + a long-chain acid anion.